{
  "term_id": "GO:0008458",
  "gene": "UniProtKB:Q9UKG9",
  "gene_symbol": "CROT",
  "gene_name": "Peroxisomal carnitine O-octanoyltransferase",
  "term_label": "carnitine O-octanoyltransferase activity"
}